regulation of extracellular matrix constituent secretion [GO:0003330] (biological process) Sources: GOC:dph, GOC:tb Definition: Any process that modulates the rate, frequency, or extent of the controlled release of molecules that form the extracellular matrix, including carbohydrates and glycoproteins by a cell or a group of cells. Subtypes: GO:0003331, GO:0003332 Relationships: is_a regulation of extracellular matrix organization [GO:1903053]; is a type of regulation of secretion by cell [GO:1903530]; regulates extracellular matrix constituent secretion [GO:0070278]